{
  "gene_name": "Cyclin-O",
  "gene_symbol": "CCNO",
  "gene": "UniProtKB:P22674",
  "term_label": "cyclin-dependent protein kinase holoenzyme complex",
  "term_id": "GO:0000307"
}